primary methylamine oxidase activity [GO:0008131] (molecular function) Definition: Catalysis of the reaction: a primary methyl amine + H2O + O2 = an aldehyde + H2O2 + NH4+. Sources: RHEA:16153 Also known as: amine oxidase activity, primary-amine:oxygen oxidoreductase (deaminating) activity, amine oxidase (copper-containing) activity, primary amine oxidase activity Relationships: is a type of oxidoreductase activity, acting on the CH-NH2 group of donors, oxygen as acceptor [GO:0016641] Subtypes: L-amino-acid oxidase activity [GO:0001716], D-amino-acid oxidase activity [GO:0003884], GO:0018527